{
  "gene_symbol": "FES",
  "gene": "UniProtKB:P07332",
  "gene_name": "Tyrosine-protein kinase Fes_Fps",
  "term_label": "protein tyrosine kinase activity",
  "term_id": "GO:0004713"
}